actin filament network formation [GO:0051639] (biological process) Sources: GOC:ai Also known as: actin gel biosynthesis, actin gel formation Definition: The assembly of a network of actin filaments; actin filaments on different axes and with differing orientations are crosslinked together to form a mesh of filaments. Relationships: is a type of actin filament organization [GO:0007015]